{
  "gene_symbol": "SMARCD1",
  "gene": "UniProtKB:Q96GM5",
  "gene_name": "SWI_SNF-related matrix-associated actin-dependent regulator of chromatin subfamily D member 1",
  "term_label": "regulation of transcription by RNA polymerase II",
  "term_id": "GO:0006357"
}